{
  "gene": "UniProtKB:Q8NGJ0",
  "gene_symbol": "OR5A1",
  "term_id": "GO:0005549",
  "term_label": "odorant binding",
  "gene_name": "Olfactory receptor 5A1"
}